{
  "gene_name": "Kallikrein-12",
  "gene": "UniProtKB:Q9UKR0",
  "gene_symbol": "KLK12",
  "term_label": "extracellular space",
  "term_id": "GO:0005615"
}